1,2-diacylglycerol 3-glucosyltransferase activity [GO:0047228] (molecular function) Also known as: UDP-glucose-diacylglycerol glucosyltransferase activity, UDP-glucose:1,2-diacylglycerol 3-D-glucosyltransferase activity, UDP-glucose:1,2-diacylglycerol glucosyltransferase activity, UDPglucose:1,2-diacylglycerol 3-D-glucosyltransferase activity, UDPglucose:diacylglycerol glucosyltransferase activity, uridine diphosphoglucose-diacylglycerol glucosyltransferase activity Sources: RHEA:47612 Relationships: is a type of GO:0035251 Definition: Catalysis of the reaction: a 1,2-diacyl-sn-glycerol + UDP-alpha-D-glucose = a 1,2-diacyl-3-O-(alpha-D-glucopyranosyl)-sn-glycerol + H+ + UDP.